sex-chromosome dosage compensation [GO:0007549] (biological process) References: PMID:11498577, PMID:30049999, PMID:35306885 Sources: GOC:ems Also known as: dosage compensation, sex chromosome dosage compensation Subtypes: GO:0009047, GO:0009048, dosage compensation by hypoactivation of X chromosome [GO:0042464] Definition: Compensating for the variation in the unpaired sex chromosome:autosome chromosome ratios between sexes by activation or inactivation of genes on one or both of the sex chromosomes. Relationships: is a type of epigenetic regulation of gene expression [GO:0040029]